regulation of immature T cell proliferation [GO:0033083] (biological process) Relationships: is a type of regulation of T cell proliferation [GO:0042129]; regulates immature T cell proliferation [GO:0033079] Sources: GOC:add, GOC:mah Definition: Any process that modulates the frequency, rate or extent of immature T cell proliferation. Subtypes: regulation of immature T cell proliferation in thymus [GO:0033084], negative regulation of immature T cell proliferation [GO:0033087], positive regulation of immature T cell proliferation [GO:0033091]